ubiquitin-like protein peptidase activity [GO:0019783] (molecular function) Note: While ubiquitin-like proteins can be rarely linked to substrates via bonds other than isopeptide bonds, all known ubiquitin-like peptidases cleave the isopeptide bond. Subtypes: deSUMOylase activity [GO:0016929], deNEDDylase activity [GO:0019784], GO:0019785, ubiquitin-like protein-specific endopeptidase activity [GO:0070137], GO:0071567, GO:0101005 Definition: An isopeptidase activity that cleaves ubiquitin or ubiquitin-like proteins (ULP; e.g. ATG8, ISG15, NEDD8, SUMO) from target proteins. Also known as: small conjugating protein-specific isopeptidase activity, small conjugating protein-specific protease activity, ubiquitin-like hydrolase activity, ubiquitin-like protein-specific isopeptidase activity, ubiquitin-like protein-specific protease activity, ubiquitinyl-like hydrolase activity, ubiquitin-like specific protease activity, ubiquitin-like-protein-specific protease activity, ubiquitin-specific protease activity involved in negative regulation of ERAD pathway, ubiquitin-specific protease activity involved in positive regulation of ERAD pathway References: PMID:19489724 Relationships: is a type of peptidase activity [GO:0008233]